methionine decarboxylase activity [GO:0050095] (MF) Also known as: L-methionine carboxy-lyase (3-methylthiopropanamine-forming), L-methionine carboxy-lyase activity, L-methionine decarboxylase activity Relationships: is a type of GO:0016831 Sources: EC:4.1.1.57, RHEA:17757 Definition: Catalysis of the reaction: L-methionine + H+ = 3-methylthiopropanamine + CO2.